{
  "gene_symbol": "FBXO45",
  "term_id": "GO:0019005",
  "gene_name": "F-box_SPRY domain-containing protein 1",
  "term_label": "SCF ubiquitin ligase complex",
  "gene": "UniProtKB:P0C2W1"
}